secretory columnal luminar epithelial cell differentiation involved in prostate glandular acinus development [GO:0060528] (biological process) References: PMID:18977204 Sources: GOC:dph Relationships: is a type of glandular epithelial cell differentiation [GO:0002067]; is a type of GO:0060742; is part of prostate glandular acinus development [GO:0060525] Definition: The process in which a relatively unspecialized epithelial cell acquires specialized features of a secretory columnal luminar epithelial cell of the prostate.